oxaloglycolate reductase (decarboxylating) activity [GO:0047047] (molecular function) Definition: Catalysis of the reaction: glycerate + CO2 + NAD(P)+ = NAD(P)H + H+ + 2-hydroxy-3-oxosuccinate. Also known as: D-glycerate:NAD(P)+ oxidoreductase (carboxylating) Relationships: is a type of GO:0016616 Sources: EC:1.1.1.92, MetaCyc:1.1.1.92-RXN